{
  "gene_name": "Splicing factor 3A subunit 2",
  "gene_symbol": "SF3A2",
  "gene": "UniProtKB:Q15428",
  "term_id": "GO:0005686",
  "term_label": "U2 snRNP"
}